{
  "gene": "UniProtKB:O95843",
  "gene_name": "Guanylyl cyclase-activating protein 3",
  "term_id": "GO:0008048",
  "gene_symbol": "GUCA1C",
  "term_label": "calcium sensitive guanylate cyclase activator activity"
}